regulation of peripheral T cell tolerance induction [GO:0002849] (biological process) Sources: GOC:add Relationships: is a type of regulation of peripheral tolerance induction [GO:0002658]; is a type of GO:0002664; is a type of regulation of T cell mediated immunity [GO:0002709]; regulates peripheral T cell tolerance induction [GO:0002458] Definition: Any process that modulates the frequency, rate, or extent of peripheral T cell tolerance induction. Subtypes: regulation of T cell tolerance induction to tumor cell [GO:0002846], negative regulation of peripheral T cell tolerance induction [GO:0002850], positive regulation of peripheral T cell tolerance induction [GO:0002851]